{
  "term_id": "GO:0008284",
  "gene": "UniProtKB:P16234",
  "gene_symbol": "PDGFRA",
  "term_label": "positive regulation of cell population proliferation",
  "gene_name": "Platelet-derived growth factor receptor alpha"
}